{
  "gene_symbol": "PEX11G",
  "term_id": "GO:0005778",
  "gene": "UniProtKB:Q96HA9",
  "term_label": "peroxisomal membrane",
  "gene_name": "Peroxisomal membrane protein 11C"
}